{
  "term_label": "Unknown cellular component",
  "gene_name": "UDP-glucuronosyltransferase 2B7",
  "gene_symbol": "UGT2B7",
  "term_id": "UNKNOWN:0003",
  "gene": "UniProtKB:P16662"
}